{
  "term_label": "microtubule binding",
  "gene_symbol": "KIF20A",
  "gene_name": "Kinesin-like protein KIF20A",
  "gene": "UniProtKB:O95235",
  "term_id": "GO:0008017"
}